{
  "gene": "UniProtKB:P78371",
  "term_label": "protein folding",
  "gene_symbol": "CCT2",
  "gene_name": "T-complex protein 1 subunit beta",
  "term_id": "GO:0006457"
}